{
  "term_label": "DNA integration",
  "gene_name": "Histone-lysine N-methyltransferase SETMAR",
  "term_id": "GO:0015074",
  "gene_symbol": "SETMAR",
  "gene": "UniProtKB:Q53H47"
}